{
  "gene": "UniProtKB:Q96KX1",
  "term_id": "UNKNOWN:0003",
  "gene_name": "Uncharacterized protein C4orf36",
  "gene_symbol": "C4orf36",
  "term_label": "Unknown cellular component"
}